{
  "term_id": "GO:0051028",
  "gene_symbol": "FXR1",
  "gene": "UniProtKB:P51114",
  "gene_name": "RNA-binding protein FXR1",
  "term_label": "mRNA transport"
}